{
  "gene": "UniProtKB:Q8TD43",
  "gene_symbol": "TRPM4",
  "term_id": "GO:0005227",
  "term_label": "calcium-activated cation channel activity",
  "gene_name": "Transient receptor potential cation channel subfamily M member 4"
}